{
  "term_label": "ubiquitin-like ligase-substrate adaptor activity",
  "term_id": "GO:1990756",
  "gene_symbol": "KLHL12",
  "gene": "UniProtKB:Q53G59",
  "gene_name": "Kelch-like protein 12"
}